{
  "gene_symbol": "ZC3HAV1",
  "gene_name": "Zinc finger CCCH-type antiviral protein 1",
  "term_label": "positive regulation of mRNA catabolic process",
  "gene": "UniProtKB:Q7Z2W4",
  "term_id": "GO:0061014"
}